{
  "term_label": "extracellular matrix organization",
  "gene_name": "Collagen alpha-1(IV) chain",
  "term_id": "GO:0030198",
  "gene_symbol": "COL4A1",
  "gene": "UniProtKB:P02462"
}